{
  "gene_symbol": "PNLIP",
  "term_label": "lipoprotein lipase activity",
  "gene": "UniProtKB:P16233",
  "term_id": "GO:0004465",
  "gene_name": "Pancreatic triacylglycerol lipase"
}